{
  "gene_symbol": "H2BC1",
  "term_label": "nucleus",
  "gene": "UniProtKB:Q96A08",
  "term_id": "GO:0005634",
  "gene_name": "Histone H2B type 1-A"
}